zinc ion binding [GO:0008270] (molecular function) Relationships: is a type of transition metal ion binding [GO:0046914] Also known as: Zn binding, zinc binding Definition: Binding to a zinc ion (Zn). Sources: GOC:ai